{
  "gene_name": "Protein RCC2",
  "term_label": "chromosome passenger complex localization to kinetochore",
  "term_id": "GO:0072356",
  "gene_symbol": "RCC2",
  "gene": "UniProtKB:Q9P258"
}